{
  "gene_name": "Olfactory receptor 52R1",
  "gene_symbol": "OR52R1",
  "term_id": "UNKNOWN:0002",
  "gene": "UniProtKB:Q8NGF1",
  "term_label": "Unknown biological process"
}